{
  "term_label": "positive regulation of neuron apoptotic process",
  "term_id": "GO:0043525",
  "gene": "UniProtKB:P49840",
  "gene_symbol": "GSK3A",
  "gene_name": "Glycogen synthase kinase-3 alpha"
}